{
  "gene_symbol": "CIMAP1A",
  "term_label": "cytoskeleton",
  "gene_name": "Outer dense fiber protein 3",
  "term_id": "GO:0005856",
  "gene": "UniProtKB:Q96PU9"
}